{
  "term_id": "GO:0007015",
  "gene": "UniProtKB:Q6ZRI8",
  "gene_symbol": "ARHGAP36",
  "term_label": "actin filament organization",
  "gene_name": "Rho GTPase-activating protein 36"
}